{
  "gene_name": "Reticulophagy regulator 3",
  "term_id": "UNKNOWN:0002",
  "gene": "UniProtKB:Q86VR2",
  "gene_symbol": "RETREG3",
  "term_label": "Unknown biological process"
}